{
  "gene_name": "T cell receptor alpha joining 6 (Fragment)",
  "gene": "UniProtKB:A0A075B6Z3",
  "gene_symbol": "TRAJ6",
  "term_label": "Unknown molecular function",
  "term_id": "UNKNOWN:0001"
}